{
  "term_id": "GO:0051082",
  "gene": "UniProtKB:P25685",
  "gene_name": "DnaJ homolog subfamily B member 1",
  "gene_symbol": "DNAJB1",
  "term_label": "unfolded protein binding"
}